complement component C4b receptor activity [GO:0001861] (molecular function) Definition: Combining with the C4b product of the classical complement cascade and transmitting the signal from one side of the membrane to the other to initiate a change in cell activity. Sources: GOC:add, GOC:signaling, ISBN:0781735149 Relationships: is a type of opsonin receptor activity [GO:0001847]; is a type of complement receptor activity [GO:0004875]; has part complement component C4b binding [GO:0001855]